{
  "term_id": "GO:0007165",
  "gene": "UniProtKB:Q32ZL2",
  "gene_symbol": "PLPPR5",
  "gene_name": "Phospholipid phosphatase-related protein type 5",
  "term_label": "signal transduction"
}